{
  "gene": "UniProtKB:P54105",
  "term_label": "pICln-Sm protein complex",
  "term_id": "GO:0034715",
  "gene_name": "Methylosome subunit pICln",
  "gene_symbol": "CLNS1A"
}